mesonephric renal vesicle induction [GO:0061294] (biological process) Sources: GOC:mtg_kidney_jan10 Relationships: is a type of regulation of mesonephros development [GO:0061217]; is a type of renal vesicle induction [GO:0072034]; positively regulates mesonephric renal vesicle formation [GO:0061262] Definition: Signaling at short range between cells of the ureteric bud terminus and the kidney mesenchyme that positively regulates the formation of the mesonephric renal vesicle.